{
  "gene_symbol": "CD96",
  "gene": "UniProtKB:P40200",
  "term_id": "UNKNOWN:0001",
  "gene_name": "T-cell surface protein tactile",
  "term_label": "Unknown molecular function"
}